{
  "gene_name": "Reticulon-4 receptor",
  "term_id": "GO:0009897",
  "gene": "UniProtKB:Q9BZR6",
  "term_label": "external side of plasma membrane",
  "gene_symbol": "RTN4R"
}